positive regulation of interleukin-24 production [GO:0032748] (biological process) Definition: Any process that activates or increases the frequency, rate, or extent of interleukin-24 production. Also known as: positive regulation of IL-24 production, up regulation of interleukin-24 production, up-regulation of interleukin-24 production, upregulation of interleukin-24 production, activation of interleukin-24 production, positive regulation of interleukin-24 biosynthetic process, stimulation of interleukin-24 production Relationships: is a type of positive regulation of cytokine production [GO:0001819]; is a type of regulation of interleukin-24 production [GO:0032668]; positively regulates GO:0032628 Sources: GOC:mah